{
  "term_label": "neuropeptide signaling pathway",
  "gene": "UniProtKB:Q5JQD4",
  "gene_symbol": "PYY3",
  "term_id": "GO:0007218",
  "gene_name": "Putative peptide YY-3"
}